{
  "term_label": "dendrite",
  "gene_symbol": "EPHB3",
  "gene_name": "Ephrin type-B receptor 3",
  "term_id": "GO:0030425",
  "gene": "UniProtKB:P54753"
}